{
  "term_id": "GO:0070588",
  "gene_symbol": "TRPM8",
  "term_label": "calcium ion transmembrane transport",
  "gene": "UniProtKB:Q7Z2W7",
  "gene_name": "Transient receptor potential cation channel subfamily M member 8"
}